{
  "gene_symbol": "RDH14",
  "term_id": "UNKNOWN:0003",
  "term_label": "Unknown cellular component",
  "gene": "UniProtKB:Q9HBH5",
  "gene_name": "Retinol dehydrogenase 14"
}